positive regulation of leukocyte tethering or rolling [GO:1903238] (BP) Definition: Any process that activates or increases the frequency, rate or extent of leukocyte tethering or rolling. Also known as: up regulation of leukocyte tethering or rolling, up-regulation of leukocyte tethering or rolling, upregulation of leukocyte tethering or rolling, activation of leukocyte tethering or rolling Relationships: is_a regulation of leukocyte tethering or rolling [GO:1903236]; is a type of positive regulation of leukocyte adhesion to vascular endothelial cell [GO:1904996]; positively regulates GO:0050901 References: PMID:18308860 Sources: GOC:TermGenie, GOC:als, GO_REF:0000058